{
  "term_id": "GO:0000812",
  "gene_name": "Craniofacial development protein 1",
  "gene": "UniProtKB:Q9UEE9",
  "term_label": "Swr1 complex",
  "gene_symbol": "CFDP1"
}